FMRP-CYFIP1 complex [GO:0160209] (cellular component) References: PMID:18805096, PMID:28183735 Relationships: is a type of intracellular protein-containing complex [GO:0140535] Definition: A protein-containing complex that contains the fragile X mental retardation protein (FMRP) and cytoplasmic FMRP Interacting protein 1 (CYIFIP1), and is capable of inhibiting translation initiation by binding to the eIF4F complex.